{
  "gene_name": "Guanine nucleotide-binding protein G(z) subunit alpha",
  "term_label": "heterotrimeric G-protein complex",
  "gene": "UniProtKB:P19086",
  "term_id": "GO:0005834",
  "gene_symbol": "GNAZ"
}